{
  "term_id": "GO:0031463",
  "gene_name": "BTB_POZ domain-containing protein KCTD2",
  "gene": "UniProtKB:Q14681",
  "gene_symbol": "KCTD2",
  "term_label": "Cul3-RING ubiquitin ligase complex"
}